{
  "term_id": "GO:0031267",
  "gene": "UniProtKB:Q14C86",
  "term_label": "small GTPase binding",
  "gene_name": "GTPase-activating protein and VPS9 domain-containing protein 1",
  "gene_symbol": "GAPVD1"
}